{
  "gene_name": "Prostaglandin D2 receptor 2",
  "gene": "UniProtKB:Q9Y5Y4",
  "term_label": "neuron projection",
  "gene_symbol": "PTGDR2",
  "term_id": "GO:0043005"
}